{
  "term_label": "plasma membrane",
  "gene_name": "Angiopoietin-1 receptor",
  "gene_symbol": "TEK",
  "gene": "UniProtKB:Q02763",
  "term_id": "GO:0005886"
}